heparin proteoglycan catabolic process [GO:0030211] (biological process) Definition: The chemical reactions and pathways resulting in the breakdown of heparin proteoglycans, which consist of a core protein linked to a heparin glycosaminoglycan. The heparin chain is composed of the repeating disaccharide unit beta-(1,4)-N-acetyl-D-glucosamine-alpha-(1,4)-hexuronic acid, the former being either sulfated or deacetylated on its amino group as well as sulfated on one of its hydroxyl groups and the latter being a mixture of sulfated and nonsulfated D-glucuronic and L-iduronic acids. Heparin is similar to heparan sulfate but it contains more N-sulfate and O-sulfate groups. References: PMID:35536982 Also known as: heparin breakdown, heparin catabolism, heparin degradation, heparan sulfate catabolic process Relationships: is a type of proteoglycan catabolic process [GO:0030167]; is a type of GO:0030202